{
  "gene_symbol": "RASAL1",
  "gene_name": "RasGAP-activating-like protein 1",
  "term_id": "GO:1902531",
  "term_label": "regulation of intracellular signal transduction",
  "gene": "UniProtKB:O95294"
}